{
  "gene_name": "Transcription factor MafA",
  "gene": "UniProtKB:Q8NHW3",
  "term_label": "DNA-binding transcription factor activity, RNA polymerase II-specific",
  "term_id": "GO:0000981",
  "gene_symbol": "MAFA"
}